{
  "gene_name": "Amelotin",
  "term_label": "odontogenesis of dentin-containing tooth",
  "gene_symbol": "AMTN",
  "term_id": "GO:0042475",
  "gene": "UniProtKB:Q6UX39"
}